{
  "gene_symbol": "NSFL1C",
  "gene_name": "NSFL1 cofactor p47",
  "term_id": "GO:0043130",
  "gene": "UniProtKB:Q9UNZ2",
  "term_label": "ubiquitin binding"
}